{
  "term_label": "ciliary base",
  "gene": "UniProtKB:Q6ZVS7",
  "gene_symbol": "CFAP144P1",
  "term_id": "GO:0097546",
  "gene_name": "Protein FAM183BP"
}